{
  "term_label": "RNA polymerase II cis-regulatory region sequence-specific DNA binding",
  "term_id": "GO:0000978",
  "gene_symbol": "KLF9",
  "gene_name": "Krueppel-like factor 9",
  "gene": "UniProtKB:Q13886"
}